{
  "gene": "UniProtKB:O60939",
  "gene_name": "Sodium channel subunit beta-2",
  "gene_symbol": "SCN2B",
  "term_label": "plasma membrane",
  "term_id": "GO:0005886"
}